{
  "gene_name": "Protein ABHD11",
  "gene_symbol": "ABHD11",
  "term_label": "mitochondrion",
  "gene": "UniProtKB:Q8NFV4",
  "term_id": "GO:0005739"
}